stress-induced premature senescence [GO:0090400] (biological process) Also known as: SIPS Definition: A cellular senescence process associated with the dismantling of a cell as a response to environmental factors such as hydrogen peroxide or X-rays. Subtypes: oxidative stress-induced premature senescence [GO:0090403] Sources: GOC:BHF Relationships: is a type of GO:0090398